{
  "gene_name": "Junctophilin-2",
  "term_label": "plasma membrane",
  "gene_symbol": "JPH2",
  "term_id": "GO:0005886",
  "gene": "UniProtKB:Q9BR39"
}